positive regulation of sorocarp spore cell differentiation [GO:1901263] (biological process) Relationships: is a type of positive regulation of cell differentiation [GO:0045597]; is a type of regulation of sorocarp spore cell differentiation [GO:1901261]; positively regulates sorocarp spore cell differentiation [GO:0044671] Also known as: up regulation of sorocarp spore cell differentiation, up-regulation of sorocarp spore cell differentiation, upregulation of sorocarp spore cell differentiation, activation of sorocarp spore cell differentiation Sources: GOC:TermGenie, GOC:rjd Definition: Any process that activates or increases the frequency, rate or extent of sorocarp spore cell differentiation.